{
  "gene_symbol": "HLA-A",
  "gene": "UniProtKB:P04439",
  "term_id": "GO:0009897",
  "gene_name": "HLA class I histocompatibility antigen, A alpha chain",
  "term_label": "external side of plasma membrane"
}